{
  "gene_symbol": "GLCCI1",
  "term_id": "UNKNOWN:0002",
  "gene_name": "Glucocorticoid-induced transcript 1 protein",
  "term_label": "Unknown biological process",
  "gene": "UniProtKB:Q86VQ1"
}